{
  "gene_name": "Mesenteric estrogen-dependent adipogenesis protein",
  "term_label": "Unknown molecular function",
  "gene_symbol": "MEDAG",
  "gene": "UniProtKB:Q5VYS4",
  "term_id": "UNKNOWN:0001"
}